maintenance of root meristem identity [GO:0010078] (biological process) Definition: The process in which an organism retains a population of root meristem cells, preventing the commitment of all stem cell progeny to a differentiated cell fate. Relationships: is a type of maintenance of meristem identity [GO:0010074]; is part of GO:0010015 Sources: GOC:dph, GOC:tb